{
  "term_id": "GO:0000724",
  "gene_name": "Bifunctional 3'-5' exonuclease_ATP-dependent helicase WRN",
  "term_label": "double-strand break repair via homologous recombination",
  "gene": "UniProtKB:Q14191",
  "gene_symbol": "WRN"
}